positive regulation of protein localization to cell tip [GO:1903068] (biological process) References: PMID:24554432 Sources: GOC:TermGenie, GO_REF:0000058 Relationships: is a type of GO:1903066; is_a positive regulation of protein localization [GO:1903829]; positively regulates protein localization to cell tip [GO:1990151] Also known as: positive regulation of protein localisation to cell tip, up regulation of protein localisation to cell tip, up regulation of protein localization to cell tip, up-regulation of protein localisation to cell tip, up-regulation of protein localization to cell tip, upregulation of protein localisation to cell tip, upregulation of protein localization to cell tip, activation of protein localisation to cell tip, activation of protein localization to cell tip Definition: Any process that activates or increases the frequency, rate or extent of protein localization to cell tip.